regulation of natural killer cell cytokine production [GO:0002727] (biological process) Definition: Any process that modulates the frequency, rate, or extent of natural killer cell cytokine production. Relationships: is a type of GO:0002715; is a type of regulation of cytokine production involved in immune response [GO:0002718]; regulates natural killer cell cytokine production [GO:0002370] Also known as: regulation of NK cell cytokine production Subtypes: negative regulation of natural killer cell cytokine production [GO:0002728], positive regulation of natural killer cell cytokine production [GO:0002729] Sources: GOC:add